{
  "term_id": "UNKNOWN:0001",
  "term_label": "Unknown molecular function",
  "gene_name": "FERM and PDZ domain-containing protein 1",
  "gene_symbol": "FRMPD1",
  "gene": "UniProtKB:Q5SYB0"
}